{
  "term_id": "GO:0000976",
  "gene_name": "Zinc finger protein 112",
  "gene_symbol": "ZNF112",
  "term_label": "transcription cis-regulatory region binding",
  "gene": "UniProtKB:Q9UJU3"
}